defense response to nematode [GO:0002215] (biological process) Definition: A response to protect an organism from a directly detected or perceived external threat from a nematode or nematodes, which results in restriction of damage to the organism attacked or prevention/recovery from the infection caused by the attack. References: PMID:11516579, PMID:14506883 Sources: GOC:add Also known as: physiological defense response to nematode Relationships: is a type of defense response [GO:0006952]; is a type of GO:0051707 Subtypes: behavioral defense response to nematode [GO:0002212]